{
  "gene": "UniProtKB:A0A0A0MTA7",
  "term_label": "Unknown molecular function",
  "gene_symbol": "TRBJ2-1",
  "term_id": "UNKNOWN:0001",
  "gene_name": "T cell receptor beta joining 2-1"
}